{
  "term_label": "negative regulation of DNA-templated transcription",
  "gene": "UniProtKB:C9JLR9",
  "term_id": "GO:0045892",
  "gene_name": "Zinc finger translocation-associated protein",
  "gene_symbol": "ZFTA"
}